mannitol-1-phosphatase activity [GO:0050084] (molecular function) Also known as: D-mannitol-1-phosphate phosphohydrolase activity, mannitol-1-phosphate phosphatase activity Sources: EC:3.1.3.22, RHEA:19537 Relationships: is a type of phosphatase activity [GO:0016791] Definition: Catalysis of the reaction: D-mannitol 1-phosphate + H2O = D-mannitol + 2 H+ + phosphate.